PAMP receptor decoy activity [GO:0140320] (molecular function) Also known as: pathogen-associated molecular pattern receptor decoy activity, pattern recognition receptor decoy activity Relationships: is a type of receptor decoy activity [GO:0140319] References: PMID:20724636 Definition: Binding and sequestering PAMP ligands in order to prevent them from binding and activating to the host PAMP receptor. Usually this activity is encoded by a symbiont or a pathogen to prevent activation of the host innate immune response.